{
  "term_label": "Unknown cellular component",
  "term_id": "UNKNOWN:0003",
  "gene": "UniProtKB:B4DX44",
  "gene_symbol": "ZNF736",
  "gene_name": "Zinc finger protein 736"
}